{
  "term_label": "Unknown biological process",
  "gene_name": "Ankyrin repeat domain-containing protein 63",
  "gene": "UniProtKB:C9JTQ0",
  "term_id": "UNKNOWN:0002",
  "gene_symbol": "ANKRD63"
}